regulation of platelet formation [GO:1905219] (biological process) Also known as: regulation of platelet extrusion Relationships: is a type of GO:0022604; is_a regulation of myeloid cell differentiation [GO:0045637]; RO_0002211 platelet formation [GO:0030220] References: PMID:10606160 Sources: GOC:TermGenie, GO_REF:0000058 Definition: Any process that modulates the frequency, rate or extent of platelet formation. Subtypes: negative regulation of platelet formation [GO:1905220], positive regulation of platelet formation [GO:1905221]